{
  "term_id": "GO:0006508",
  "gene": "UniProtKB:P48052",
  "term_label": "proteolysis",
  "gene_name": "Carboxypeptidase A2",
  "gene_symbol": "CPA2"
}